polyubiquitinated protein transport [GO:0070844] (biological process) References: PMID:14675537 Sources: GOC:BHF, GOC:mah Relationships: is a type of intracellular protein transport [GO:0006886] Also known as: polyubiquitylated protein transport Definition: The directed movement of polyubiquitinated proteins in a cell, including the movement of proteins between specific compartments or structures within a cell. Subtypes: GO:0070845